{
  "gene_symbol": "AK1",
  "term_id": "GO:0004017",
  "gene": "UniProtKB:P00568",
  "term_label": "AMP kinase activity",
  "gene_name": "Adenylate kinase isoenzyme 1"
}